{
  "gene": "UniProtKB:P56962",
  "term_id": "GO:0006906",
  "gene_symbol": "STX17",
  "gene_name": "Syntaxin-17",
  "term_label": "vesicle fusion"
}